positive regulation of viral budding via host ESCRT complex [GO:1903774] (biological process) Definition: Any process that activates or increases the frequency, rate or extent of viral budding via host ESCRT complex. Also known as: up regulation of viral budding via host ESCRT complex, up-regulation of viral budding via host ESCRT complex, upregulation of viral budding via host ESCRT complex, activation of viral budding via host ESCRT complex, activation of viral budding through the ESCRT machinery, positive regulation of viral budding through the ESCRT machinery, up regulation of viral budding through the ESCRT machinery, up-regulation of viral budding through the ESCRT machinery, upregulation of viral budding through the ESCRT machinery References: PMID:24878737 Sources: GOC:TermGenie, GOC:als, GO_REF:0000058 Relationships: is a type of GO:1903772; is_a positive regulation of viral life cycle [GO:1903902]; positively regulates viral budding via host ESCRT complex [GO:0039702]